IkappaB kinase complex [GO:0008385] (cellular component) Also known as: IKK complex, heterotrimeric IKK complex, trimeric IKK complex Definition: A trimeric protein complex that phosphorylates inhibitory-kappaB (I-kappaB) proteins. The complex is composed of two kinase subunits (alpha and beta) and a regulatory gamma subunit (also called NEMO). In a resting state, NF-kappaB dimers are bound to inhibitory IKB proteins, sequestering NF-kappaB in the cytoplasm. Phosphorylation of I-kappaB targets I-kappaB for ubiquitination and proteasomal degradation, thus releasing the NF-kappaB dimers, which can translocate to the nucleus to bind DNA and regulate transcription. Relationships: is a type of serine/threonine protein kinase complex [GO:1902554]; BFO_0000050 GO:0005829 References: PMID:12055104, PMID:20300203 Sources: GOC:bf, GOC:ma